positive regulation of neutrophil mediated killing of gram-negative bacterium [GO:0070963] (biological process) Relationships: is a type of regulation of neutrophil mediated killing of gram-negative bacterium [GO:0070951]; is a type of positive regulation of neutrophil mediated killing of bacterium [GO:0070962]; positively regulates neutrophil-mediated killing of gram-negative bacterium [GO:0070945] Sources: GOC:add, GOC:mah Also known as: up regulation of neutrophil mediated killing of gram-negative bacterium, up-regulation of neutrophil mediated killing of gram-negative bacterium, upregulation of neutrophil mediated killing of gram-negative bacterium, activation of neutrophil mediated killing of gram-negative bacterium, stimulation of neutrophil mediated killing of gram-negative bacterium Definition: Any process that increases the frequency, rate or extent of the directed killing of a gram-negative bacterium by a neutrophil.